{
  "gene_name": "Uncharacterized protein C9orf40",
  "gene": "UniProtKB:Q8IXQ3",
  "term_label": "Unknown cellular component",
  "term_id": "UNKNOWN:0003",
  "gene_symbol": "C9orf40"
}